{
  "gene_symbol": "ABCB11",
  "gene": "UniProtKB:O95342",
  "gene_name": "Bile salt export pump",
  "term_label": "transmembrane transport",
  "term_id": "GO:0055085"
}